{
  "gene_name": "Argininosuccinate lyase",
  "term_label": "cytosol",
  "gene": "UniProtKB:P04424",
  "gene_symbol": "ASL",
  "term_id": "GO:0005829"
}